{
  "gene_name": "Keratin, type II cytoskeletal 78",
  "gene": "UniProtKB:Q8N1N4",
  "term_label": "keratinization",
  "term_id": "GO:0031424",
  "gene_symbol": "KRT78"
}